2-hydroxyquinoline 8-monooxygenase activity [GO:0033766] (molecular function) Sources: EC:1.14.13.61, RHEA:22080 Relationships: is a type of oxidoreductase activity, acting on paired donors, with incorporation or reduction of molecular oxygen, NAD(P)H as one donor, and incorporation of one atom of oxygen [GO:0016709] Definition: Catalysis of the reaction: H+ + NADH + O2 + quinolin-2-ol = H2O + NAD+ + quinoline-2,8-diol. Also known as: 2-oxo-1,2-dihydroquinoline 8-monooxygenase activity, quinolin-2(1H)-one,NADH:oxygen oxidoreductase (8-oxygenating) activity